{
  "gene_symbol": "NARS2",
  "term_label": "mitochondrion",
  "gene_name": "Probable asparagine--tRNA ligase, mitochondrial",
  "term_id": "GO:0005739",
  "gene": "UniProtKB:Q96I59"
}